{
  "gene_symbol": "MAFIP",
  "term_label": "Unknown molecular function",
  "gene": "UniProtKB:Q8WZ33",
  "term_id": "UNKNOWN:0001",
  "gene_name": "MaFF-interacting protein"
}